{
  "term_label": "intracellular signal transduction",
  "term_id": "GO:0035556",
  "gene_name": "Serine_threonine-protein kinase 32C",
  "gene_symbol": "STK32C",
  "gene": "UniProtKB:Q86UX6"
}